{
  "gene": "UniProtKB:Q9NWF9",
  "gene_symbol": "RNF216",
  "term_label": "Unknown molecular function",
  "term_id": "UNKNOWN:0001",
  "gene_name": "E3 ubiquitin-protein ligase RNF216"
}